{
  "gene_name": "Centrosomal protein of 85 kDa",
  "gene": "UniProtKB:Q6P2H3",
  "gene_symbol": "CEP85",
  "term_id": "GO:0005813",
  "term_label": "centrosome"
}